{
  "gene_name": "Small G protein signaling modulator 1",
  "term_id": "UNKNOWN:0003",
  "term_label": "Unknown cellular component",
  "gene_symbol": "SGSM1",
  "gene": "UniProtKB:Q2NKQ1"
}